{
  "gene_name": "Zinc finger CCCH domain-containing protein 7B",
  "gene_symbol": "ZC3H7B",
  "term_id": "GO:0035198",
  "term_label": "miRNA binding",
  "gene": "UniProtKB:Q9UGR2"
}